carbon-carbon lyase activity [GO:0016830] (molecular function) Subtypes: GO:0003913, 3,4-dihydroxy-2-butanone-4-phosphate synthase activity [GO:0008686], tryptophanase activity [GO:0009034], GO:0016831, aldehyde-lyase activity [GO:0016832], oxo-acid-lyase activity [GO:0016833], benzylsuccinate synthase activity [GO:0018805], 2-iminoacetate synthase activity [GO:0036355], tyrosine phenol-lyase activity [GO:0050371], GTP 3',8'-cyclase activity [GO:0061798], phosphomethylpyrimidine synthase activity [GO:0070284], aldehyde oxygenase (deformylating) activity [GO:0071771], long-chain fatty aldehyde oxidative decarbonylase activity [GO:0160238] Also known as: other carbon-carbon lyase activity Sources: GOC:jl Relationships: is a type of lyase activity [GO:0016829] Definition: Catalysis of the cleavage of C-C bonds by other means than by hydrolysis or oxidation, or conversely adding a group to a double bond.